Schwann cell proliferation [GO:0014010] (biological process) Sources: GOC:ef, ISBN:0878932585 Relationships: is a type of glial cell proliferation [GO:0014009] Subtypes: Schwann cell proliferation involved in axon regeneration [GO:0014011] Definition: The multiplication or reproduction of Schwann cells, resulting in the expansion of their population. Schwann cells are a type of glial cell in the peripheral nervous system. Regulation: regulated by regulation of Schwann cell proliferation [GO:0010624]; positively regulated by positive regulation of Schwann cell proliferation [GO:0010625]; negatively regulated by negative regulation of Schwann cell proliferation [GO:0010626]